{
  "term_label": "Unknown cellular component",
  "gene_name": "1-phosphatidylinositol 4,5-bisphosphate phosphodiesterase epsilon-1",
  "term_id": "UNKNOWN:0003",
  "gene_symbol": "PLCE1",
  "gene": "UniProtKB:Q9P212"
}